{
  "term_label": "Unknown cellular component",
  "term_id": "UNKNOWN:0003",
  "gene": "UniProtKB:P35453",
  "gene_name": "Homeobox protein Hox-D13",
  "gene_symbol": "HOXD13"
}